{
  "gene_symbol": "DDX24",
  "gene": "UniProtKB:Q9GZR7",
  "term_label": "Unknown biological process",
  "gene_name": "ATP-dependent RNA helicase DDX24",
  "term_id": "UNKNOWN:0002"
}